response to peptide [GO:1901652] (biological process) Sources: GOC:TermGenie, GOC:pr Relationships: is a type of response to chemical [GO:0042221] Definition: Any process that results in a change in state or activity of a cell or an organism (in terms of movement, secretion, enzyme production, gene expression, etc.) as a result of a peptide stimulus. Subtypes: response to cytokine [GO:0034097], cellular response to peptide [GO:1901653]